{
  "term_label": "RNA polymerase II cis-regulatory region sequence-specific DNA binding",
  "gene_name": "Tissue-resident T-cell transcription regulator protein ZNF683",
  "term_id": "GO:0000978",
  "gene_symbol": "ZNF683",
  "gene": "UniProtKB:Q8IZ20"
}